{
  "gene_name": "Nuclear factor NF-kappa-B p100 subunit",
  "term_label": "Unknown cellular component",
  "gene": "UniProtKB:Q00653",
  "gene_symbol": "NFKB2",
  "term_id": "UNKNOWN:0003"
}